mBAF complex [GO:0140091] (cellular component) Relationships: is a type of GO:0070603 References: PMID:11175787, PMID:12620226, PMID:15525990, PMID:8804307, PMID:8895581 Sources: GO:bhm Definition: A muscle cell-specific SWI/SNF-type complex that contains eight to fourteen proteins, including both conserved (core) and nonconserved components; contains the ATPase product of either the SMARCA4/BAF190A/BRG1 gene, the mammalian ortholog of the yeast SNF2 gene, or the SMARCA2/BAF190B/BRM gene, the mammalian ortholog of the Drosophila brm (brahma) gene, or an ortholog of either of these genes, and the muscle-specific product of the DPF3/BAF45C gene or an ortholog thereof. Also known as: muscle-specific BAF complex, muscle-specific SWI/SNF complex, muscle-type BAF complex, muscle-type SWI/SNF complex